{
  "gene_name": "Transmembrane protein 134",
  "term_id": "UNKNOWN:0003",
  "gene_symbol": "TMEM134",
  "term_label": "Unknown cellular component",
  "gene": "UniProtKB:Q9H6X4"
}